{
  "term_label": "cytoplasm",
  "gene_symbol": "ARHGAP40",
  "gene_name": "Rho GTPase-activating protein 40",
  "term_id": "GO:0005737",
  "gene": "UniProtKB:Q5TG30"
}